{
  "gene": "UniProtKB:B0I1T2",
  "gene_name": "Unconventional myosin-Ig",
  "term_label": "actin filament organization",
  "term_id": "GO:0007015",
  "gene_symbol": "MYO1G"
}